{
  "term_id": "UNKNOWN:0002",
  "gene_symbol": "SPDYE17",
  "gene_name": "Putative speedy protein E17",
  "term_label": "Unknown biological process",
  "gene": "UniProtKB:P0DUD2"
}